cell differentiation involved in mesonephros development [GO:0061208] (biological process) Definition: The process in which relatively unspecialized cells acquire specialized structural and/or functional features that characterize the cells of the mesonephros as it progresses from its formation to the mature state. Sources: GOC:mtg_kidney_jan10 Subtypes: GO:0061207, GO:0061223, mesenchymal stem cell differentiation involved in mesonephric nephron morphogenesis [GO:0061239], mesonephric glomerular epithelial cell differentiation [GO:0061250], mesonephric mesangial cell differentiation [GO:0061260], mesenchymal to epithelial transition involved in mesonephros morphogenesis [GO:0061261], mesonephric nephron tubule epithelial cell differentiation [GO:0061265], mesonephric interstitial fibroblast differentiation [GO:0061266], mesenchymal stem cell differentiation involved in metanephric nephron morphogenesis [GO:0072281] Relationships: is a type of GO:0061005; is part of mesonephros development [GO:0001823]